complement component C3dg binding [GO:0001853] (molecular function) Definition: Binding to a C3dg product of the complement cascade. Sources: GOC:add, ISBN:0781735149 Relationships: is a type of complement binding [GO:0001848]